{
  "gene": "UniProtKB:Q8N6M8",
  "term_label": "positive regulation of acrosome reaction",
  "term_id": "GO:2000344",
  "gene_name": "IQ domain-containing protein F1",
  "gene_symbol": "IQCF1"
}